{
  "gene": "UniProtKB:O75879",
  "term_id": "GO:0050567",
  "gene_symbol": "GATB",
  "gene_name": "Glutamyl-tRNA(Gln) amidotransferase subunit B, mitochondrial",
  "term_label": "glutaminyl-tRNA synthase (glutamine-hydrolyzing) activity"
}